{
  "term_label": "cell-matrix adhesion",
  "term_id": "GO:0007160",
  "gene_name": "Vitronectin",
  "gene": "UniProtKB:P04004",
  "gene_symbol": "VTN"
}